adrenomedullin receptor signaling pathway [GO:1990410] (biological process) Relationships: is a type of calcitonin family receptor signaling pathway [GO:0097646] Note: An example of a protein that could be annotated to this term is CALCRL in human (Q16602) in PMID:10882736. Definition: The series of molecular signals initiated by an extracellular adrenomedullin combining with a dimeric adrenomedullin receptor on the surface of the target cell. References: PMID:10882736 Sources: GOC:bhm Also known as: AM receptor signaling pathway